{
  "term_label": "RNA endonuclease activity",
  "term_id": "GO:0004521",
  "gene": "UniProtKB:Q6P5S7",
  "gene_name": "Ribonuclease kappa",
  "gene_symbol": "RNASEK"
}